{
  "gene_symbol": "GSE1",
  "term_id": "UNKNOWN:0003",
  "gene": "UniProtKB:Q14687",
  "gene_name": "Genetic suppressor element 1",
  "term_label": "Unknown cellular component"
}